diacetylchitobiose deacetylase activity [GO:0052773] (molecular function) Relationships: is a type of GO:0016811 Also known as: N,N'-diacetylchitobiose deacetylase (nonreducing end) References: PMID:15136574, PMID:16232910, PMID:16736587 Sources: RHEA:62168 Definition: Catalysis of the reaction: H2O + N,N'-diacetylchitobiose = acetate + beta-D-glucosaminyl-(1->4)-N-acetyl-D-glucosamine. Note: In this reaction N,N'-diacetylchitobiose is deacetylated at the non-reducing residue to produce 2-acetamido-4-O-(2-amino-2-deoxy-beta-D-glucopyranosyl)-2-deoxy-D-glucose (GlcN-GlcNAc). This is in contrast to EC:3.5.1.105 in which N,N'-diacetylchitobiose is deacetylated at the reducing residue to produce 4-O-(N-acetyl-beta-D-glucosaminyl)-D-glucosamine (GlcNAc-GlcN). For the latter reaction, see GO:0036311.